{
  "term_label": "meiotic spindle organization",
  "gene_name": "Tubulin gamma-1 chain",
  "gene_symbol": "TUBG1",
  "gene": "UniProtKB:P23258",
  "term_id": "GO:0000212"
}